{
  "gene": "UniProtKB:Q49A88",
  "gene_name": "Coiled-coil domain-containing protein 14",
  "gene_symbol": "CCDC14",
  "term_label": "Unknown molecular function",
  "term_id": "UNKNOWN:0001"
}